protein localization to Golgi membrane [GO:1903292] (biological process) Relationships: is a type of protein localization to Golgi apparatus [GO:0034067]; is a type of protein localization to membrane [GO:0072657] Also known as: protein localisation in Golgi membrane, protein localisation to Golgi membrane, protein localization in Golgi membrane Definition: A process in which a protein is transported to, or maintained in, a location within a Golgi membrane. References: PMID:11378902 Sources: GOC:TermGenie, GO_REF:0000087